nuclear body organization [GO:0030575] (BP) Relationships: is a type of nucleus organization [GO:0006997] Also known as: nuclear body organisation, nuclear body organization and biogenesis Subtypes: Cajal body organization [GO:0030576], Lands organization [GO:0030577], GO:0030578, nuclear speck organization [GO:0035063], GO:0140167, nuclear dicing body assembly [GO:1904258] Definition: A process that is carried out at the cellular level which results in the assembly, arrangement of constituent parts, or disassembly of any of the extra-nucleolar nuclear domains usually visualized by confocal microscopy and fluorescent antibodies to specific proteins. Sources: GOC:dph, GOC:jl, GOC:mah